cellular response to methyl methanesulfonate [GO:0072703] (biological process) Relationships: is a type of response to methyl methanesulfonate [GO:0072702]; is a type of cellular response to oxygen-containing compound [GO:1901701] Definition: Any process that results in a change in state or activity of a cell (in terms of movement, secretion, enzyme production, gene expression, etc.) as a result of a methyl methanesulfonate (MMS) stimulus. Sources: GOC:mah Also known as: cellular response to MMS